{
  "gene_name": "Uncharacterized protein CXorf66",
  "gene_symbol": "CXorf66",
  "gene": "UniProtKB:Q5JRM2",
  "term_id": "UNKNOWN:0002",
  "term_label": "Unknown biological process"
}